{
  "gene": "UniProtKB:Q9HB71",
  "gene_symbol": "CACYBP",
  "gene_name": "Calcyclin-binding protein",
  "term_label": "ubiquitin protein ligase binding",
  "term_id": "GO:0031625"
}